{
  "gene": "UniProtKB:Q9BZY9",
  "term_id": "GO:0045087",
  "gene_name": "E3 ubiquitin-protein ligase TRIM31",
  "term_label": "innate immune response",
  "gene_symbol": "TRIM31"
}